regulation of outer hair cell apoptotic process [GO:1905585] (biological process) Relationships: is a type of regulation of neuron apoptotic process [GO:0043523]; regulates outer hair cell apoptotic process [GO:1905584] Also known as: regulation of cochlear outer hair cell apoptotic process, regulation of cochlear outer hair cell apoptosis, regulation of outer hair cell apoptosis References: PMID:24472721 Sources: GOC:TermGenie, GO_REF:0000058 Definition: Any process that modulates the frequency, rate or extent of outer hair cell apoptotic process. Subtypes: negative regulation of outer hair cell apoptotic process [GO:1905586], positive regulation of outer hair cell apoptotic process [GO:1905587]